{
  "term_id": "UNKNOWN:0002",
  "gene": "UniProtKB:Q6ICH7",
  "gene_symbol": "ASPHD2",
  "term_label": "Unknown biological process",
  "gene_name": "Aspartate beta-hydroxylase domain-containing protein 2"
}